{
  "gene_symbol": "ANAPC5",
  "term_label": "anaphase-promoting complex",
  "term_id": "GO:0005680",
  "gene": "UniProtKB:Q9UJX4",
  "gene_name": "Anaphase-promoting complex subunit 5"
}